{
  "gene_symbol": "TSHZ3",
  "term_label": "nucleus",
  "gene_name": "Teashirt homolog 3",
  "gene": "UniProtKB:Q63HK5",
  "term_id": "GO:0005634"
}